response to gonadotropin-releasing hormone [GO:0097210] (biological process) Subtypes: cellular response to gonadotropin-releasing hormone [GO:0097211] Relationships: is a type of response to peptide hormone [GO:0043434] References: PMID:15976007 Sources: GOC:yaf Definition: Any process that results in a change in state or activity of a cell or an organism (in terms of movement, secretion, enzyme production, gene expression, etc.) as a result of a gonadotropin-releasing hormone stimulus. Gonadotropin-releasing hormone (GnRH) is a peptide hormone responsible for the release of follicle-stimulating hormone (FSH) and luteinizing hormone (LH) from the anterior pituitary. GnRH is synthesized and released by the hypothalamus. Also known as: response to GnRH